{
  "gene_name": "Sharpin",
  "gene": "UniProtKB:Q9H0F6",
  "term_id": "GO:0097039",
  "term_label": "protein linear polyubiquitination",
  "gene_symbol": "SHARPIN"
}